{
  "gene_symbol": "MFSD5",
  "gene": "UniProtKB:Q6N075",
  "term_label": "Unknown cellular component",
  "term_id": "UNKNOWN:0003",
  "gene_name": "Molybdate-anion transporter"
}